D-aspartate import across plasma membrane [GO:0070779] (biological process) Regulation: regulated by regulation of D-aspartate import across plasma membrane [GO:0140215]; negatively regulated by negative regulation of D-aspartate import across plasma membrane [GO:0140216]; positively regulated by positive regulation of D-aspartate import across plasma membrane [GO:0140217] Also known as: D-aspartate import, D-aspartate import into cell, D-aspartate uptake Relationships: is a type of D-aspartate transmembrane transport [GO:0070777]; is a type of GO:0089718 Definition: The directed import of D-aspartate from the extracellular region across the plasma membrane and into the cytosol. References: PMID:7914198